regulation of cellulosome assembly [GO:1900503] (biological process) Sources: GOC:TermGenie, GOC:mengo_curators Subtypes: negative regulation of cellulosome assembly [GO:1900504], positive regulation of cellulosome assembly [GO:1900505] Relationships: is a type of GO:1902115; RO_0002211 cellulosome assembly [GO:0044575] Definition: Any process that modulates the frequency, rate or extent of cellulosome assembly.